{
  "gene_symbol": "PRDM11",
  "term_id": "GO:0045165",
  "gene_name": "PR domain-containing protein 11",
  "gene": "UniProtKB:Q9NQV5",
  "term_label": "cell fate commitment"
}